pyruvate decarboxylase activity [GO:0004737] (molecular function) Relationships: is a type of GO:0016831 Sources: EC:4.1.1.1 Definition: Catalysis of the reaction: a 2-oxo acid = an aldehyde + CO2. Also known as: 2-oxo-acid carboxy-lyase (aldehyde-forming), 2-oxo-acid carboxy-lyase activity, alpha-carboxylase activity, alpha-ketoacid carboxylase activity, pyruvic decarboxylase activity